{
  "gene_name": "Prickle-like protein 4",
  "term_label": "muscle structure development",
  "gene_symbol": "PRICKLE4",
  "term_id": "GO:0061061",
  "gene": "UniProtKB:Q2TBC4"
}